{
  "gene_name": "Tubulin beta 8B",
  "term_label": "mitotic cell cycle",
  "term_id": "GO:0000278",
  "gene": "UniProtKB:A6NNZ2",
  "gene_symbol": "TUBB8B"
}